{
  "term_id": "GO:0016020",
  "gene_symbol": "VPS39",
  "gene": "UniProtKB:Q96JC1",
  "term_label": "membrane",
  "gene_name": "Vam6_Vps39-like protein"
}